actinorhodin biosynthetic process [GO:1901112] (biological process) Definition: The chemical reactions and pathways resulting in the formation of actinorhodin. Also known as: actinorhodin anabolism, actinorhodin biosynthesis, actinorhodin formation, actinorhodin synthesis Relationships: is a type of dicarboxylic acid biosynthetic process [GO:0043650] Sources: GOC:TermGenie, GOC:yaf, UniPathway:UPA00173